{
  "term_label": "Unknown molecular function",
  "gene_name": "Lymphocyte antigen 6D",
  "gene_symbol": "LY6D",
  "term_id": "UNKNOWN:0001",
  "gene": "UniProtKB:Q14210"
}